{
  "gene_symbol": "LCMT1",
  "term_label": "cytosol",
  "gene_name": "Leucine carboxyl methyltransferase 1",
  "gene": "UniProtKB:Q9UIC8",
  "term_id": "GO:0005829"
}